{
  "term_id": "GO:1902936",
  "gene_name": "Clavesin-1",
  "term_label": "phosphatidylinositol bisphosphate binding",
  "gene_symbol": "CLVS1",
  "gene": "UniProtKB:Q8IUQ0"
}